{
  "term_label": "Unknown biological process",
  "gene": "UniProtKB:P80188",
  "term_id": "UNKNOWN:0002",
  "gene_symbol": "LCN2",
  "gene_name": "Neutrophil gelatinase-associated lipocalin"
}